{
  "term_id": "UNKNOWN:0001",
  "gene_symbol": "DRC1",
  "term_label": "Unknown molecular function",
  "gene": "UniProtKB:Q96MC2",
  "gene_name": "Dynein regulatory complex protein 1"
}